{
  "gene_name": "F-box and leucine-rich repeat protein 13",
  "gene": "UniProtKB:Q8NEE6",
  "term_id": "UNKNOWN:0001",
  "gene_symbol": "FBXL13",
  "term_label": "Unknown molecular function"
}